cyclic nucleotide binding [GO:0030551] (molecular function) Sources: GOC:ai Definition: Binding to a cyclic nucleotide, a nucleotide in which the phosphate group is in diester linkage to two positions on the sugar residue. Relationships: is a type of nucleotide binding [GO:0000166] Subtypes: GO:0030552, cGMP binding [GO:0030553], cyclic-di-GMP binding [GO:0035438], GO:0140702, cyclic-di-AMP binding [GO:0180001]